{
  "term_label": "kinesin complex",
  "gene": "UniProtKB:Q12840",
  "gene_symbol": "KIF5A",
  "gene_name": "Kinesin heavy chain isoform 5A",
  "term_id": "GO:0005871"
}